{
  "gene": "UniProtKB:Q9Y6N3",
  "gene_name": "Calcium-activated chloride channel regulator family member 3",
  "term_id": "UNKNOWN:0003",
  "gene_symbol": "CLCA3P",
  "term_label": "Unknown cellular component"
}